{
  "gene": "UniProtKB:Q9NYG2",
  "gene_symbol": "ZDHHC3",
  "gene_name": "Palmitoyltransferase ZDHHC3",
  "term_id": "GO:0005794",
  "term_label": "Golgi apparatus"
}